adherens junction organization [GO:0034332] (biological process) Definition: A process that is carried out at the cellular level which results in the assembly, arrangement of constituent parts, or disassembly of an adherens junction. An adherens junction is a cell-cell junction composed of the epithelial cadherin-catenin complex at which the cytoplasmic face of the plasma membrane is attached to actin filaments. Sources: GOC:aruk, GOC:bc, GOC:dph, GOC:jl, GOC:mah Also known as: adherens junction organisation Subtypes: GO:0034333, adherens junction maintenance [GO:0034334], adherens junction disassembly [GO:0120179] Relationships: is a type of cell-cell junction organization [GO:0045216] Regulation: regulated by regulation of adherens junction organization [GO:1903391]; negatively regulated by GO:1903392; positively regulated by positive regulation of adherens junction organization [GO:1903393]